{
  "term_id": "GO:0005634",
  "gene_name": "BAG family molecular chaperone regulator 1",
  "gene": "UniProtKB:Q99933",
  "term_label": "nucleus",
  "gene_symbol": "BAG1"
}